{
  "gene": "UniProtKB:P40337",
  "term_label": "Unknown biological process",
  "gene_name": "von Hippel-Lindau disease tumor suppressor",
  "term_id": "UNKNOWN:0002",
  "gene_symbol": "VHL"
}